{
  "term_label": "DNA-binding transcription factor activity, RNA polymerase II-specific",
  "gene": "UniProtKB:A6NI15",
  "term_id": "GO:0000981",
  "gene_symbol": "MSGN1",
  "gene_name": "Mesogenin-1"
}